interleukin-12 binding [GO:0019972] (molecular function) Subtypes: interleukin-12 beta subunit binding [GO:0042163], interleukin-12 alpha subunit binding [GO:0042164] Definition: Binding to interleukin-12. Relationships: is a type of GO:0019955 Also known as: IL-12 binding Sources: GOC:jl